{
  "gene_symbol": "GABRA4",
  "gene_name": "Gamma-aminobutyric acid receptor subunit alpha-4",
  "term_label": "dendrite membrane",
  "term_id": "GO:0032590",
  "gene": "UniProtKB:P48169"
}